{
  "term_label": "nucleus",
  "gene_name": "Zinc fingers and homeoboxes protein 2",
  "gene": "UniProtKB:Q9Y6X8",
  "term_id": "GO:0005634",
  "gene_symbol": "ZHX2"
}